{
  "term_label": "Unknown molecular function",
  "gene": "UniProtKB:P0DMU8",
  "gene_symbol": "CT45A5",
  "gene_name": "Cancer_testis antigen family 45 member A5",
  "term_id": "UNKNOWN:0001"
}